regulation of violaceol II biosynthetic process [GO:1900716] (biological process) Definition: Any process that modulates the frequency, rate or extent of violaceol II biosynthetic process. Relationships: is a type of regulation of secondary metabolite biosynthetic process [GO:1900376]; regulates violaceol II biosynthetic process [GO:1900593] Also known as: regulation of violaceol II anabolism, regulation of violaceol II biosynthesis, regulation of violaceol II formation, regulation of violaceol II synthesis Subtypes: GO:1900717, GO:1900718 Sources: GOC:TermGenie, GOC:di